{
  "term_id": "GO:0016020",
  "term_label": "membrane",
  "gene_name": "Potassium voltage-gated channel subfamily KQT member 2",
  "gene_symbol": "KCNQ2",
  "gene": "UniProtKB:O43526"
}